{
  "gene_symbol": "SHB",
  "gene_name": "SH2 domain-containing adapter protein B",
  "term_id": "GO:0001784",
  "gene": "UniProtKB:Q15464",
  "term_label": "phosphotyrosine residue binding"
}